{
  "gene": "UniProtKB:P78318",
  "term_id": "GO:0005829",
  "gene_name": "Immunoglobulin-binding protein 1",
  "gene_symbol": "IGBP1",
  "term_label": "cytosol"
}